interleukin-3-mediated signaling pathway [GO:0038156] (biological process) Sources: GOC:nhn, GOC:signaling Relationships: is a type of cytokine-mediated signaling pathway [GO:0019221] Also known as: IL-3-mediated signaling pathway, interleukin-3-mediated signalling pathway Definition: The series of molecular signals initiated by interleukin-3 binding to its receptor on the surface of a target cell, and ending with the regulation of a downstream cellular process, e.g. transcription.